{
  "term_label": "nucleus",
  "term_id": "GO:0005634",
  "gene": "UniProtKB:P52756",
  "gene_symbol": "RBM5",
  "gene_name": "RNA-binding protein 5"
}